{
  "gene": "UniProtKB:Q9BRK0",
  "gene_symbol": "REEP2",
  "term_label": "endoplasmic reticulum membrane",
  "term_id": "GO:0005789",
  "gene_name": "Receptor expression-enhancing protein 2"
}